{
  "gene_name": "Interleukin-12 receptor subunit beta-1",
  "gene": "UniProtKB:P42701",
  "term_id": "GO:0019221",
  "gene_symbol": "IL12RB1",
  "term_label": "cytokine-mediated signaling pathway"
}